{
  "term_label": "Unknown cellular component",
  "term_id": "UNKNOWN:0003",
  "gene_symbol": "LINC00612",
  "gene_name": "Putative uncharacterized protein encoded by LINC00612",
  "gene": "UniProtKB:Q8N6U2"
}